{
  "gene_name": "Alpha-actinin-2",
  "gene": "UniProtKB:P35609",
  "term_label": "Z disc",
  "gene_symbol": "ACTN2",
  "term_id": "GO:0030018"
}